hindbrain maturation [GO:0021578] (biological process) Sources: GOC:cls, GOC:dgh, GOC:dph, GOC:jid, GO_REF:0000021 Relationships: is a type of anatomical structure maturation [GO:0071695]; is part of central nervous system maturation [GO:0021626]; is part of hindbrain development [GO:0030902] Definition: A developmental process, independent of morphogenetic (shape) change, that is required for the hindbrain to attain its fully functional state. The hindbrain is the region consisting of the medulla, pons and cerebellum. Areas of the hindbrain control motor and autonomic functions.